{
  "gene_name": "Transmembrane protein 45A",
  "term_label": "Unknown molecular function",
  "gene_symbol": "TMEM45A",
  "gene": "UniProtKB:Q9NWC5",
  "term_id": "UNKNOWN:0001"
}